{
  "gene_name": "Cadherin-2",
  "gene": "UniProtKB:P19022",
  "term_label": "cell-cell junction assembly",
  "term_id": "GO:0007043",
  "gene_symbol": "CDH2"
}